{
  "term_label": "RNA splicing",
  "gene": "UniProtKB:Q9Y2W2",
  "gene_symbol": "WBP11",
  "gene_name": "WW domain-binding protein 11",
  "term_id": "GO:0008380"
}